ascus epiplasm [GO:0072324] (CC) Relationships: is a type of cellular anatomical structure [GO:0110165] Note: Note that this term is an is_a child of 'cell part' because the epiplasm is extracellular to the spore (each of which is a cell) but within the ascus structure, and originated from cytoplasm. Definition: Ascus cytoplasm that is not packaged into ascospores. Sources: DOI:10.1016/S0953-7562(96)80057-8, GOC:mcc